{
  "gene_name": "PAXIP1-associated glutamate-rich protein 1",
  "gene_symbol": "PAGR1",
  "term_label": "nuclear estrogen receptor binding",
  "gene": "UniProtKB:Q9BTK6",
  "term_id": "GO:0030331"
}